{
  "gene_name": "p53 and DNA damage-regulated protein 1",
  "gene": "UniProtKB:Q9NUG6",
  "term_id": "UNKNOWN:0003",
  "gene_symbol": "PDRG1",
  "term_label": "Unknown cellular component"
}